{
  "gene": "UniProtKB:P42768",
  "gene_name": "Actin nucleation-promoting factor WAS",
  "gene_symbol": "WAS",
  "term_label": "Unknown biological process",
  "term_id": "UNKNOWN:0002"
}